negative regulation of smooth muscle cell proliferation [GO:0048662] (biological process) Definition: Any process that stops, prevents or reduces the rate or extent of smooth muscle cell proliferation. Sources: CL:0000192, GOC:ebc Also known as: down regulation of smooth muscle cell proliferation, down-regulation of smooth muscle cell proliferation, downregulation of smooth muscle cell proliferation, negative regulation of SMC proliferation, inhibition of smooth muscle cell proliferation Relationships: is_a negative regulation of cell population proliferation [GO:0008285]; is a type of GO:0048660; negatively regulates smooth muscle cell proliferation [GO:0048659] Subtypes: negative regulation of vascular associated smooth muscle cell proliferation [GO:1904706]